{
  "term_label": "extracellular matrix structural constituent conferring tensile strength",
  "gene_symbol": "COL13A1",
  "gene": "UniProtKB:Q5TAT6",
  "gene_name": "Collagen alpha-1(XIII) chain",
  "term_id": "GO:0030020"
}